{
  "gene_name": "Transcriptional regulator ATRX",
  "term_id": "GO:0006338",
  "gene": "UniProtKB:P46100",
  "term_label": "chromatin remodeling",
  "gene_symbol": "ATRX"
}